maintenance of spindle location [GO:0051687] (biological process) Sources: GOC:ai, GOC:dph, GOC:tb Definition: Any process in which the spindle is maintained in a specific location within a cell and prevented from moving elsewhere. Relationships: is a type of spindle localization [GO:0051653]; is a type of maintenance of organelle location [GO:0051657] Also known as: maintenance of spindle localization